{
  "term_id": "UNKNOWN:0001",
  "term_label": "Unknown molecular function",
  "gene_name": "DPEP2 neighbor protein",
  "gene": "UniProtKB:A0A0U1RQF7",
  "gene_symbol": "DPEP2NB"
}